{
  "term_label": "nucleus",
  "gene_name": "Serine_threonine-protein phosphatase 6 regulatory subunit 1",
  "gene": "UniProtKB:Q9UPN7",
  "gene_symbol": "PPP6R1",
  "term_id": "GO:0005634"
}